{
  "term_label": "Unknown molecular function",
  "gene": "UniProtKB:Q96AT1",
  "term_id": "UNKNOWN:0001",
  "gene_name": "Uncharacterized protein KIAA1143",
  "gene_symbol": "KIAA1143"
}